{
  "term_id": "UNKNOWN:0001",
  "gene": "UniProtKB:Q9NVM9",
  "gene_name": "Integrator complex subunit 13",
  "term_label": "Unknown molecular function",
  "gene_symbol": "INTS13"
}